{
  "term_id": "GO:0005794",
  "gene_symbol": "WDR44",
  "term_label": "Golgi apparatus",
  "gene_name": "WD repeat-containing protein 44",
  "gene": "UniProtKB:Q5JSH3"
}